{
  "gene_symbol": "MAP3K5",
  "term_label": "neuron apoptotic process",
  "gene": "UniProtKB:Q99683",
  "term_id": "GO:0051402",
  "gene_name": "Mitogen-activated protein kinase kinase kinase 5"
}